{
  "gene_name": "Myc proto-oncogene protein",
  "term_label": "DNA-binding transcription factor activity, RNA polymerase II-specific",
  "gene_symbol": "MYC",
  "term_id": "GO:0000981",
  "gene": "UniProtKB:P01106"
}